{
  "gene": "UniProtKB:O43395",
  "term_id": "GO:0046540",
  "term_label": "U4/U6 x U5 tri-snRNP complex",
  "gene_name": "U4_U6 small nuclear ribonucleoprotein Prp3",
  "gene_symbol": "PRPF3"
}